{
  "gene": "UniProtKB:Q5XKE5",
  "gene_symbol": "KRT79",
  "term_label": "intermediate filament organization",
  "term_id": "GO:0045109",
  "gene_name": "Keratin, type II cytoskeletal 79"
}